{
  "term_id": "GO:0097009",
  "gene_symbol": "PPARD",
  "gene_name": "Peroxisome proliferator-activated receptor delta",
  "term_label": "energy homeostasis",
  "gene": "UniProtKB:Q03181"
}